translation elongation factor activity [GO:0003746] (molecular function) Relationships: is a type of translation factor activity [GO:0180051]; is part of translational elongation [GO:0006414] Sources: ISBN:0198506732 Definition: Functions in chain elongation during polypeptide synthesis at the ribosome.